{
  "term_id": "UNKNOWN:0002",
  "gene": "UniProtKB:Q6ZRH7",
  "gene_name": "Cation channel sperm-associated auxiliary subunit gamma",
  "term_label": "Unknown biological process",
  "gene_symbol": "CATSPERG"
}